{
  "term_id": "GO:0045944",
  "gene": "UniProtKB:Q92793",
  "gene_name": "CREB-binding protein",
  "gene_symbol": "CREBBP",
  "term_label": "positive regulation of transcription by RNA polymerase II"
}